{
  "gene_name": "Minor histocompatibility antigen H13",
  "term_id": "GO:0098554",
  "term_label": "cytoplasmic side of endoplasmic reticulum membrane",
  "gene_symbol": "HM13",
  "gene": "UniProtKB:Q8TCT9"
}